{
  "term_label": "regulation of transcription by RNA polymerase II",
  "gene_symbol": "MED7",
  "gene": "UniProtKB:O43513",
  "term_id": "GO:0006357",
  "gene_name": "Mediator of RNA polymerase II transcription subunit 7"
}